{
  "term_label": "Unknown biological process",
  "gene_name": "Proteoglycan 4",
  "gene_symbol": "PRG4",
  "gene": "UniProtKB:Q92954",
  "term_id": "UNKNOWN:0002"
}